regulation of monocyte chemotactic protein-1 production [GO:0071637] (biological process) Subtypes: negative regulation of monocyte chemotactic protein-1 production [GO:0071638], positive regulation of monocyte chemotactic protein-1 production [GO:0071639] Sources: GOC:mah Definition: Any process that modulates the frequency, rate, or extent of production of monocyte chemotactic protein-1. Also known as: regulation of CCL2 production, regulation of MCP-1 production Relationships: is a type of regulation of chemokine production [GO:0032642]; regulates monocyte chemotactic protein-1 production [GO:0071605]